{
  "term_id": "GO:0008009",
  "gene_symbol": "CCL4",
  "term_label": "chemokine activity",
  "gene_name": "C-C motif chemokine 4",
  "gene": "UniProtKB:P13236"
}